positive regulation of neutrophil activation [GO:1902565] (biological process) References: PMID:17588661 Sources: GOC:TermGenie Relationships: is a type of positive regulation of leukocyte activation [GO:0002696]; is a type of regulation of neutrophil activation [GO:1902563]; positively regulates neutrophil activation [GO:0042119] Also known as: up regulation of neutrophil activation, up-regulation of neutrophil activation, upregulation of neutrophil activation, activation of neutrophil activation Definition: Any process that activates or increases the frequency, rate or extent of neutrophil activation.